{
  "gene_symbol": "TRGJP2",
  "term_id": "UNKNOWN:0003",
  "gene": "UniProtKB:A0A0A0MT84",
  "gene_name": "T cell receptor gamma joining P2 (Fragment)",
  "term_label": "Unknown cellular component"
}